{
  "gene_symbol": "AGAP11",
  "gene_name": "Arf-GAP with GTPase, ANK repeat and PH domain-containing protein 11",
  "term_label": "GTPase activator activity",
  "term_id": "GO:0005096",
  "gene": "UniProtKB:Q8TF27"
}